{
  "term_label": "Unknown cellular component",
  "gene_symbol": "TMEM164",
  "gene": "UniProtKB:Q5U3C3",
  "term_id": "UNKNOWN:0003",
  "gene_name": "Transmembrane protein 164"
}